{
  "gene_name": "Uncharacterized protein CXorf38",
  "gene_symbol": "CXorf38",
  "term_id": "UNKNOWN:0001",
  "gene": "UniProtKB:Q8TB03",
  "term_label": "Unknown molecular function"
}